{
  "gene_name": "Puromycin-sensitive aminopeptidase-like protein",
  "term_id": "GO:0070006",
  "gene": "UniProtKB:A6NEC2",
  "gene_symbol": "NPEPPSL1",
  "term_label": "metalloaminopeptidase activity"
}